fungal-type cell wall polysaccharide biosynthetic process [GO:0051278] (biological process) Subtypes: galactoxylomannan biosynthetic process [GO:0062191], beta-1,2-oligomannoside biosynthetic process [GO:0070136], fungal-type cell wall (1->3)-alpha-glucan biosynthetic process [GO:0070600], fungal-type cell wall beta-glucan biosynthetic process [GO:0070880], galactosaminogalactan biosynthetic process [GO:0106218] Relationships: is a type of cell wall polysaccharide biosynthetic process [GO:0070592]; is a type of fungal-type cell wall polysaccharide metabolic process [GO:0071966]; is part of fungal-type cell wall biogenesis [GO:0009272] Also known as: cell wall polysaccharide anabolism, cell wall polysaccharide formation, cell wall polysaccharide synthesis, chitin- and beta-glucan-containing cell wall polysaccharide biosynthetic process Definition: The chemical reactions and pathways resulting in the formation of the polysaccharides which make up the fungal-type cell wall. Sources: GOC:ai, GOC:mtg_sensu